{
  "term_label": "plasma membrane",
  "gene_symbol": "HTR3B",
  "gene_name": "5-hydroxytryptamine receptor 3B",
  "term_id": "GO:0005886",
  "gene": "UniProtKB:O95264"
}